{
  "gene": "UniProtKB:Q9H0U3",
  "term_id": "UNKNOWN:0001",
  "gene_name": "Magnesium transporter protein 1",
  "gene_symbol": "MAGT1",
  "term_label": "Unknown molecular function"
}